{
  "term_id": "UNKNOWN:0002",
  "term_label": "Unknown biological process",
  "gene": "UniProtKB:Q96NG3",
  "gene_name": "Outer dynein arm-docking complex subunit 4",
  "gene_symbol": "ODAD4"
}